{
  "term_label": "Unknown molecular function",
  "gene": "UniProtKB:O95147",
  "term_id": "UNKNOWN:0001",
  "gene_name": "Dual specificity protein phosphatase 14",
  "gene_symbol": "DUSP14"
}